3-methylbutanoyl-CoA dehydrogenase activity [GO:0008470] (MF) Also known as: isovaleryl-CoA dehydrogenase activity, 3-methylbutanoyl-CoA:(acceptor) oxidoreductase activity, 3-methylbutanoyl-CoA:acceptor oxidoreductase activity, isovaleroyl-coenzyme A dehydrogenase activity, isovaleryl-coenzyme A dehydrogenase activity Definition: Catalysis of the reaction: 3-methylbutanoyl-CoA + H+ + oxidized [electron-transfer flavoprotein] = 3-methyl-(2E)-butenoyl-CoA + reduced [electron-transfer flavoprotein]. Relationships: is a type of short-chain fatty acyl-CoA dehydrogenase activity [GO:0016937] References: PMID:25450250, PMID:7640268 Sources: RHEA:12276